{
  "gene_name": "Sphingosine kinase 2",
  "term_label": "cytoplasm",
  "gene_symbol": "SPHK2",
  "term_id": "GO:0005737",
  "gene": "UniProtKB:Q9NRA0"
}